{
  "term_id": "GO:0030672",
  "gene_name": "Synapsin-3",
  "gene_symbol": "SYN3",
  "gene": "UniProtKB:O14994",
  "term_label": "synaptic vesicle membrane"
}